{
  "gene_symbol": "NRXN2",
  "gene_name": "Neurexin-2",
  "term_label": "adult behavior",
  "term_id": "GO:0030534",
  "gene": "UniProtKB:Q9P2S2"
}